low-affinity sulfate:proton symporter activity [GO:0009676] (molecular function) Definition: Enables the transfer of a solute or solutes from one side of a membrane to the other according to the reaction: sulfate(out) + H+(out) = sulfate(in) + H+(in). In low-affinity transport the transporter is able to bind the solute only if it is present at very high concentrations. References: PMID:7568135 Sources: GOC:mah Also known as: low affinity sulfate:hydrogen symporter activity, low affinity sulfate:proton symporter activity, low affinity sulphate:hydrogen symporter activity Relationships: is a type of sulfate:proton symporter activity [GO:0008512]